{
  "gene_symbol": "CTXND1",
  "term_label": "Unknown cellular component",
  "gene_name": "Cortexin domain-containing 1 protein",
  "gene": "UniProtKB:A0A1B0GTU2",
  "term_id": "UNKNOWN:0003"
}